{
  "term_id": "GO:0031507",
  "gene_symbol": "H2AB3",
  "gene": "UniProtKB:P0C5Z0",
  "gene_name": "Histone H2A-Bbd type 2_3",
  "term_label": "heterochromatin formation"
}